{
  "term_id": "GO:0000978",
  "gene": "UniProtKB:Q9UI36",
  "gene_name": "Dachshund homolog 1",
  "gene_symbol": "DACH1",
  "term_label": "RNA polymerase II cis-regulatory region sequence-specific DNA binding"
}